cotyledon development [GO:0048825] (biological process) Definition: The process whose specific outcome is the progression of the cotyledon over time, from its formation to the mature structure. The cotyledon is the modified leaf (seed leaf), found as part of the embryo in plant seeds. It is involved in either storage or absorption of food reserves. Dicotyledonous seeds contain two cotyledons, while monocotyledonous seeds contain only one. The cotyledons may appear above ground and show photosynthetic activity in the seedling. Relationships: is a type of embryo development ending in seed dormancy [GO:0009793]; is a type of leaf development [GO:0048366] Sources: GOC:devbiol, GOC:tb, PO:0020030